{
  "gene_symbol": "MYO15A",
  "gene": "UniProtKB:Q9UKN7",
  "term_label": "cytoplasm",
  "gene_name": "Unconventional myosin-XV",
  "term_id": "GO:0005737"
}